{
  "term_label": "transcription regulator complex",
  "gene_symbol": "NFATC4",
  "term_id": "GO:0005667",
  "gene": "UniProtKB:Q14934",
  "gene_name": "Nuclear factor of activated T-cells, cytoplasmic 4"
}